{
  "term_id": "GO:0034727",
  "gene_symbol": "ATG13",
  "gene_name": "Autophagy-related protein 13",
  "gene": "UniProtKB:O75143",
  "term_label": "piecemeal microautophagy of the nucleus"
}